{
  "gene_name": "Bifunctional glutamate_proline--tRNA ligase",
  "term_id": "GO:0017101",
  "gene": "UniProtKB:P07814",
  "gene_symbol": "EPRS1",
  "term_label": "aminoacyl-tRNA synthetase multienzyme complex"
}